cytosine metabolic process [GO:0019858] (biological process) Definition: The chemical reactions and pathways involving cytosine, 4-amino-2-hydroxypyrimidine, a pyrimidine derivative that is one of the five main bases found in nucleic acids; it occurs widely in cytidine derivatives. Relationships: is a type of GO:0006206 Subtypes: cytosine catabolic process [GO:0006209] Also known as: cytosine metabolism Sources: GOC:ai